{
  "gene_symbol": "STIM1",
  "gene": "UniProtKB:Q13586",
  "term_id": "GO:0005783",
  "term_label": "endoplasmic reticulum",
  "gene_name": "Stromal interaction molecule 1"
}